{
  "gene_symbol": "HLA-DQB2",
  "gene_name": "HLA class II histocompatibility antigen, DQ beta 2 chain",
  "term_label": "MHC class II protein complex",
  "term_id": "GO:0042613",
  "gene": "UniProtKB:P05538"
}